purine nucleoside bisphosphate catabolic process [GO:0034034] (biological process) Definition: The chemical reactions and pathways resulting in the breakdown of a purine nucleoside bisphosphate, a compound consisting of a purine base linked to a deoxyribose or ribose sugar esterified with one phosphate group attached to each of two different hydroxyl groups on the sugar. Sources: GOC:mah, GOC:pde Also known as: purine nucleoside bisphosphate breakdown, purine nucleoside bisphosphate catabolism, purine nucleoside bisphosphate degradation Relationships: is a type of GO:0033869; is a type of purine nucleoside bisphosphate metabolic process [GO:0034032]; is a type of GO:0072523 Subtypes: purine ribonucleoside bisphosphate catabolic process [GO:0034037]